{
  "gene": "UniProtKB:Q9P0J6",
  "term_label": "Unknown molecular function",
  "term_id": "UNKNOWN:0001",
  "gene_name": "Large ribosomal subunit protein bL36m",
  "gene_symbol": "MRPL36"
}